branch elongation involved in mammary gland duct branching [GO:0060751] (BP) Subtypes: GO:0060654 Also known as: mammary gland duct branch elongation Relationships: is a type of GO:0060602; is part of branching involved in mammary gland duct morphogenesis [GO:0060444] Sources: GOC:dph Definition: The developmental growth process in which a branch of a mammary gland duct elongates.